{
  "gene_name": "Neural proliferation differentiation and control protein 1",
  "term_label": "Unknown biological process",
  "term_id": "UNKNOWN:0002",
  "gene_symbol": "NPDC1",
  "gene": "UniProtKB:Q9NQX5"
}